{
  "term_id": "GO:0005737",
  "term_label": "cytoplasm",
  "gene_symbol": "MT1A",
  "gene": "UniProtKB:P04731",
  "gene_name": "Metallothionein-1A"
}